{
  "gene": "UniProtKB:Q9UJT1",
  "gene_name": "Tubulin delta chain",
  "term_id": "GO:0005525",
  "term_label": "GTP binding",
  "gene_symbol": "TUBD1"
}